{
  "term_id": "GO:0000981",
  "term_label": "DNA-binding transcription factor activity, RNA polymerase II-specific",
  "gene_name": "Transcription factor Sp6",
  "gene": "UniProtKB:Q3SY56",
  "gene_symbol": "SP6"
}